{
  "gene_symbol": "UBIAD1",
  "term_id": "GO:0005783",
  "gene": "UniProtKB:Q9Y5Z9",
  "term_label": "endoplasmic reticulum",
  "gene_name": "UbiA prenyltransferase domain-containing protein 1"
}